Wpl/Pds5 cohesin loading/unloading complex [GO:0090695] (cellular component) Relationships: is_a SMC loading complex [GO:0032116] Definition: A eukaryotically conserved heterodimeric protein complex (comprising Wings apart-like protein and the Pds5 Armadillo repeat cohesin associated protein) involved in the loading and unloading of a cohesin complex onto DNA. References: PMID:26687354 Sources: GOC:vw